{
  "term_id": "UNKNOWN:0001",
  "gene_symbol": "SPAG16",
  "gene_name": "Sperm-associated antigen 16 protein",
  "term_label": "Unknown molecular function",
  "gene": "UniProtKB:Q8N0X2"
}